{
  "gene": "UniProtKB:A6NGB0",
  "gene_symbol": "TMEM191C",
  "term_label": "Unknown biological process",
  "gene_name": "Transmembrane protein 191C",
  "term_id": "UNKNOWN:0002"
}